{
  "term_id": "GO:0000281",
  "gene": "UniProtKB:Q53EZ4",
  "term_label": "mitotic cytokinesis",
  "gene_name": "Centrosomal protein of 55 kDa",
  "gene_symbol": "CEP55"
}